{
  "gene_name": "Acetylcholine receptor subunit epsilon",
  "gene": "UniProtKB:Q04844",
  "term_label": "monoatomic ion transmembrane transport",
  "term_id": "GO:0034220",
  "gene_symbol": "CHRNE"
}